{
  "term_label": "3-mercaptopyruvate sulfurtransferase activity",
  "gene_symbol": "MPST",
  "gene_name": "3-mercaptopyruvate sulfurtransferase",
  "term_id": "GO:0016784",
  "gene": "UniProtKB:P25325"
}